{
  "gene": "UniProtKB:Q14012",
  "term_id": "GO:0014069",
  "term_label": "postsynaptic density",
  "gene_symbol": "CAMK1",
  "gene_name": "Calcium_calmodulin-dependent protein kinase type 1"
}